{
  "gene_name": "Eukaryotic translation initiation factor 4 gamma 2",
  "gene_symbol": "EIF4G2",
  "term_label": "eukaryotic translation initiation factor 4F complex",
  "term_id": "GO:0016281",
  "gene": "UniProtKB:P78344"
}